{
  "gene_symbol": "PRR20A",
  "gene_name": "Proline-rich protein 20A",
  "term_id": "UNKNOWN:0003",
  "term_label": "Unknown cellular component",
  "gene": "UniProtKB:P86496"
}